{
  "term_label": "nucleus",
  "gene_name": "Histone chaperone ASF1A",
  "gene": "UniProtKB:Q9Y294",
  "term_id": "GO:0005634",
  "gene_symbol": "ASF1A"
}